{
  "term_label": "Unknown molecular function",
  "gene_symbol": "ASPM",
  "gene_name": "Abnormal spindle-like microcephaly-associated protein",
  "gene": "UniProtKB:Q8IZT6",
  "term_id": "UNKNOWN:0001"
}